preprophase band assembly [GO:0000913] (biological process) Relationships: is_a cell cycle process [GO:0022402]; is a type of cellular component assembly [GO:0022607]; is part of GO:0000911 Definition: The aggregation, arrangement and bonding together of a set of components to form the preprophase band, a dense band of microtubules that marks the position in the cell where cytokinesis will occur in cells that perform cytokinesis by cell plate formation. Also known as: preprophase band formation Sources: GOC:clt, GOC:mah